{
  "gene_symbol": "LRRC41",
  "gene_name": "Leucine-rich repeat-containing protein 41",
  "term_label": "Unknown molecular function",
  "gene": "UniProtKB:Q15345",
  "term_id": "UNKNOWN:0001"
}